{
  "gene": "UniProtKB:Q8TE23",
  "gene_name": "Taste receptor type 1 member 2",
  "term_id": "GO:0050916",
  "gene_symbol": "TAS1R2",
  "term_label": "sensory perception of sweet taste"
}